{
  "term_id": "GO:0031410",
  "gene_symbol": "KIAA0319",
  "gene": "UniProtKB:Q5VV43",
  "term_label": "cytoplasmic vesicle",
  "gene_name": "Dyslexia-associated protein KIAA0319"
}